{
  "gene_name": "Tumor necrosis factor alpha-induced protein 3",
  "term_label": "negative regulation of inflammatory response",
  "term_id": "GO:0050728",
  "gene_symbol": "TNFAIP3",
  "gene": "UniProtKB:P21580"
}